regulation of interleukin-6-mediated signaling pathway [GO:0070103] (biological process) Subtypes: negative regulation of interleukin-6-mediated signaling pathway [GO:0070104], positive regulation of interleukin-6-mediated signaling pathway [GO:0070105] Also known as: regulation of IL-6-mediated signaling pathway, regulation of interleukin-6-mediated signalling pathway Definition: Any process that modulates the rate, frequency or extent of an interleukin-6-mediated signaling pathway. Sources: GOC:BHF, GOC:mah Relationships: is a type of regulation of cytokine-mediated signaling pathway [GO:0001959]; RO_0002211 GO:0070102